{
  "gene_symbol": "RPL7",
  "term_id": "GO:0003723",
  "term_label": "RNA binding",
  "gene_name": "Large ribosomal subunit protein uL30",
  "gene": "UniProtKB:P18124"
}